sialic acid binding [GO:0033691] (molecular function) Sources: GOC:add, ISBN:9780721601465 Also known as: N-acetylneuraminic acid binding Relationships: is a type of carboxylic acid binding [GO:0031406]; is a type of carbohydrate derivative binding [GO:0097367] Definition: Binding to a sialic acid, a N- or O- substituted derivative of neuraminic acid, a nine carbon monosaccharide. Sialic acids often occur in polysaccharides, glycoproteins, and glycolipids in animals and bacteria.